{
  "gene_symbol": "KIF2B",
  "term_label": "microtubule",
  "gene_name": "Kinesin-like protein KIF2B",
  "term_id": "GO:0005874",
  "gene": "UniProtKB:Q8N4N8"
}